{
  "gene_name": "Transmembrane protein 139",
  "gene": "UniProtKB:Q8IV31",
  "gene_symbol": "TMEM139",
  "term_label": "Unknown biological process",
  "term_id": "UNKNOWN:0002"
}